{
  "gene_symbol": "SRPK2",
  "gene": "UniProtKB:P78362",
  "gene_name": "SRSF protein kinase 2",
  "term_id": "GO:0035556",
  "term_label": "intracellular signal transduction"
}